arylmalonate decarboxylase activity [GO:0047436] (molecular function) Also known as: 2-aryl-2-methylmalonate carboxy-lyase (2-arylpropanoate-forming), 2-aryl-2-methylmalonate carboxy-lyase activity, AMDASE, AMDase activity Relationships: is a type of carboxy-lyase activity [GO:0016831] Definition: Catalysis of the reaction: 2-aryl-2-methylmalonate + H+ = 2-arylpropionate + CO2. Sources: EC:4.1.1.76, RHEA:20513